{
  "gene": "UniProtKB:Q12834",
  "gene_name": "Cell division cycle protein 20 homolog",
  "term_label": "positive regulation of anaphase-promoting complex-dependent catabolic process",
  "gene_symbol": "CDC20",
  "term_id": "GO:1905786"
}